inorganic diphosphate phosphatase activity [GO:0004427] (molecular function) Also known as: inorganic diphosphatase activity, diphosphate phosphohydrolase activity, inorganic pyrophosphatase activity, pyrophosphate phosphohydrolase activity Sources: EC:3.6.1.1, RHEA:24576 Relationships: is a type of pyrophosphatase activity [GO:0016462] Definition: Catalysis of the reaction: diphosphate + H2O = H+ + 2 phosphate.